{
  "gene": "UniProtKB:A0A590UK83",
  "gene_name": "Small integral membrane protein 45",
  "term_id": "UNKNOWN:0003",
  "gene_symbol": "SMIM45",
  "term_label": "Unknown cellular component"
}